exocyst assembly [GO:0001927] (BP) Relationships: is a type of protein-containing complex assembly [GO:0065003]; is a type of GO:0140029; is part of vesicle docking involved in exocytosis [GO:0006904] References: PMID:9700152 Sources: GOC:hjd, Wikipedia:Exocyst Definition: The aggregation, arrangement and bonding together of various polypeptides into the exocyst complex. Regulation: regulated by regulation of exocyst assembly [GO:0001928]; negatively regulated by negative regulation of exocyst assembly [GO:0001929]; positively regulated by GO:0001930